endodermal-mesodermal cell signaling involved in heart induction [GO:0003134] (biological process) Also known as: endodermal-mesodermal cell signalling involved in heart induction Sources: GOC:mtg_heart Definition: Any process that mediates the transfer of information from endodermal cells to mesodermal cells that contributes to heart induction. Relationships: is a type of endodermal-mesodermal cell signaling [GO:0003133]; is part of heart induction [GO:0003129]